{
  "gene": "UniProtKB:Q86UY6",
  "gene_symbol": "NAA40",
  "gene_name": "N-alpha-acetyltransferase 40",
  "term_label": "histone H2A acetyltransferase activity",
  "term_id": "GO:0043998"
}